{
  "gene_symbol": "ABCC11",
  "gene": "UniProtKB:Q96J66",
  "term_label": "ABC-type transporter activity",
  "term_id": "GO:0140359",
  "gene_name": "ATP-binding cassette sub-family C member 11"
}